L-lysine fermentation [GO:0019475] (biological process) Definition: The chemical reactions and pathways resulting in the breakdown of L-lysine into other compounds, including acetate. References: PMID:21826218 Relationships: is a type of GO:0006083; is a type of GO:0019477; is a type of GO:0019665 Also known as: L-lysine breakdown to acetate, L-lysine catabolic process to butyrate and acetate, L-lysine degradation to acetate, lysine fermentation